{
  "term_label": "regulation of transcription by RNA polymerase II",
  "gene": "UniProtKB:Q9NR83",
  "gene_name": "SLC2A4 regulator",
  "gene_symbol": "SLC2A4RG",
  "term_id": "GO:0006357"
}